{
  "gene": "UniProtKB:A8MTQ0",
  "term_label": "DNA-binding transcription factor activity, RNA polymerase II-specific",
  "gene_symbol": "NOTO",
  "term_id": "GO:0000981",
  "gene_name": "Homeobox protein notochord"
}